{
  "gene": "UniProtKB:Q8TE67",
  "term_label": "Rho protein signal transduction",
  "gene_name": "Epidermal growth factor receptor kinase substrate 8-like protein 3",
  "gene_symbol": "EPS8L3",
  "term_id": "GO:0007266"
}